{
  "gene_symbol": "STX1A",
  "term_label": "SNAP receptor activity",
  "gene": "UniProtKB:Q16623",
  "term_id": "GO:0005484",
  "gene_name": "Syntaxin-1A"
}